{
  "gene": "UniProtKB:Q8IY33",
  "term_label": "small GTPase binding",
  "gene_symbol": "MICALL2",
  "gene_name": "MICAL-like protein 2",
  "term_id": "GO:0031267"
}